{
  "term_id": "GO:0006623",
  "gene_name": "Intermembrane lipid transfer protein VPS13C",
  "gene": "UniProtKB:Q709C8",
  "gene_symbol": "VPS13C",
  "term_label": "protein targeting to vacuole"
}